{
  "term_label": "Unknown molecular function",
  "gene_symbol": "SMIM47",
  "term_id": "UNKNOWN:0001",
  "gene": "UniProtKB:D0EPY3",
  "gene_name": "Small integral membrane protein 47"
}